{
  "gene_symbol": "ISL1",
  "term_id": "GO:0005634",
  "term_label": "nucleus",
  "gene": "UniProtKB:P61371",
  "gene_name": "Insulin gene enhancer protein ISL-1"
}